{
  "gene_name": "X-linked retinitis pigmentosa GTPase regulator",
  "gene_symbol": "RPGR",
  "term_label": "intraciliary transport",
  "term_id": "GO:0042073",
  "gene": "UniProtKB:Q92834"
}